{
  "term_id": "UNKNOWN:0003",
  "gene_symbol": "UBTD1",
  "gene_name": "Ubiquitin domain-containing protein 1",
  "term_label": "Unknown cellular component",
  "gene": "UniProtKB:Q9HAC8"
}